trihydroxybenzophenone synthase activity [GO:0102735] (molecular function) Definition: Catalysis of the reaction: benzoyl-CoA + 3 malonyl-CoA + 3 H+ = 2,4,6-trihydroxybenzophenone + 4 coenzyme A + 3 carbon dioxide. Sources: GOC:pz, RHEA:35143 Relationships: is a type of acyltransferase activity, transferring groups other than amino-acyl groups [GO:0016747]